trichloro-p-hydroquinone reductive dehalogenase activity [GO:0052690] (molecular function) Definition: Catalysis of the reaction: 2,3,6-trichlorohydroquinone + 2 glutathione = 2,6-dichlorohydroquinone + glutathione disulfide + HCl. References: PMID:1459949 Sources: RHEA:56832 Also known as: xenobiotic reductase activity, trichlorohydroquinone reductive dehalogenase activity, pentaerythritol tetranitrate reductase activity, tetrachlorohydroquinone reductive dehalogenase activity Relationships: is a type of oxidoreductase activity, acting on X-H and Y-H to form an X-Y bond [GO:0046992]